{
  "gene_symbol": "EYS",
  "term_label": "extracellular space",
  "gene": "UniProtKB:Q5T1H1",
  "gene_name": "Protein eyes shut homolog",
  "term_id": "GO:0005615"
}